chromoplast organization [GO:0009661] (biological process) Definition: A process that is carried out at the cellular level which results in the assembly, arrangement of constituent parts, or disassembly of the chromoplast. A chromoplast is a plastid containing pigments other than chlorophyll, usually yellow and orange carotenoid pigments. Sources: GOC:jid Also known as: chromoplast organisation, chromoplast organization and biogenesis Relationships: is_a plastid organization [GO:0009657]